viral release via suppression of host peptidoglycan biosynthetic process [GO:0039640] (biological process) Definition: The dissemination of mature viral particles from a host cell, caused by a virus stopping, preventing, or reducing peptidoglycan biosynthesis in the host organism. Peptidoglycans are any of a class of glycoconjugates found in bacterial cell walls. References: PMID:28894177 Sources: GOC:bf, GOC:bm Also known as: viral exit by cytolysis via suppression of host peptidoglycan biosynthetic process, viral release by cytolysis via suppression of host peptidoglycan biosynthetic process, cytolysis by virus via suppression of host peptidoglycan biosynthetic process Relationships: is a type of viral release from host cell by cytolysis [GO:0044659]; has part symbiont-mediated suppression of host peptidoglycan biosynthetic process [GO:0039635]